postsynapse organization [GO:0099173] (biological process) Definition: A process that is carried out at the cellular level which results in the assembly, arrangement of constituent parts, or disassembly of a postsynapse. Sources: GOC:dos Also known as: postsynapse development, postsynapse organisation, postsynapse morphogenesis, postsynapse organization and biogenesis Relationships: is a type of cellular component organization [GO:0016043]; is part of synapse organization [GO:0050808] Subtypes: GO:0097061, postsynapse assembly [GO:0099068] Regulation: regulated by regulation of postsynapse organization [GO:0099175]